{
  "term_id": "GO:0000977",
  "gene": "UniProtKB:Q96NG8",
  "gene_name": "Zinc finger protein 582",
  "gene_symbol": "ZNF582",
  "term_label": "RNA polymerase II transcription regulatory region sequence-specific DNA binding"
}